regulation of gut granule assembly [GO:1904755] (biological process) Subtypes: negative regulation of gut granule assembly [GO:1904756], GO:1904757 Relationships: is a type of GO:1902115; RO_0002211 gut granule assembly [GO:1902900] References: PMID:17535251 Sources: GOC:TermGenie, GO_REF:0000058 Definition: Any process that modulates the frequency, rate or extent of gut granule assembly. Also known as: regulation of gut granule biogenesis, regulation of gut granule formation